negative regulation of cell adhesion in ventricular zone [GO:0021804] (biological process) Definition: The process that results in the loss of attachments of a cell in the ventricular zone. References: PMID:12626695 Sources: GOC:cls, GOC:dgh, GOC:dph, GOC:jid, GO_REF:0000021 Relationships: is_a GO:0007162; is part of somal translocation [GO:0021802] Also known as: down regulation of cell adhesion in ventricular zone, down-regulation of cell adhesion in ventricular zone, downregulation of cell adhesion in ventricular zone, inhibition of cell adhesion in ventricular zone